{
  "gene_symbol": "MTOR",
  "gene": "UniProtKB:P42345",
  "gene_name": "Serine_threonine-protein kinase mTOR",
  "term_id": "GO:0031932",
  "term_label": "TORC2 complex"
}